{
  "gene_name": "DnaJ homolog subfamily C member 22",
  "term_label": "Unknown molecular function",
  "term_id": "UNKNOWN:0001",
  "gene": "UniProtKB:Q8N4W6",
  "gene_symbol": "DNAJC22"
}